{
  "term_id": "GO:0050808",
  "gene_symbol": "SNCA",
  "gene_name": "Alpha-synuclein",
  "term_label": "synapse organization",
  "gene": "UniProtKB:P37840"
}